negative regulation of mast cell activation involved in immune response [GO:0033007] (biological process) Definition: Any process that stops, prevents, or reduces the frequency, rate, or extent of mast cell activation as part of an immune response. Sources: GOC:mah Relationships: is a type of negative regulation of immune effector process [GO:0002698]; is a type of negative regulation of mast cell activation [GO:0033004]; is a type of GO:0033006; is a type of GO:0050777; negatively regulates mast cell activation involved in immune response [GO:0002279] Also known as: negative regulation of mast cell activation during immune response